{
  "term_id": "GO:0051726",
  "gene": "UniProtKB:Q8NEV1",
  "term_label": "regulation of cell cycle",
  "gene_symbol": "CSNK2A3",
  "gene_name": "Casein kinase II subunit alpha 3"
}